{
  "term_label": "phosphatidate phosphatase activity",
  "term_id": "GO:0008195",
  "gene": "UniProtKB:Q6T4P5",
  "gene_name": "Phospholipid phosphatase-related protein type 3",
  "gene_symbol": "PLPPR3"
}